{
  "term_label": "nicotinamide-nucleotide adenylyltransferase activity",
  "gene": "UniProtKB:Q9BZQ4",
  "term_id": "GO:0000309",
  "gene_name": "Nicotinamide_nicotinic acid mononucleotide adenylyltransferase 2",
  "gene_symbol": "NMNAT2"
}